{
  "term_id": "GO:0030162",
  "term_label": "regulation of proteolysis",
  "gene": "UniProtKB:Q6IQ16",
  "gene_name": "Speckle-type POZ protein-like",
  "gene_symbol": "SPOPL"
}